N-acetyllactosaminide 3-alpha-galactosyltransferase activity [GO:0047276] (molecular function) Definition: Catalysis of the reaction: beta-D-galactosyl-(1,4)-beta-N-acetyl-D-glucosaminyl-R + UDP-galactose = alpha-D-galactosyl-(1,3)-beta-D-galactosyl-(1,4)-beta-N-acetyl-D-glucosaminyl-R + UDP. Sources: EC:2.4.1.87, RHEA:13013 Also known as: N-acetyllactosaminide alpha-1,3-galactosyltransferase activity, beta-galactosyl-N-acetylglucosaminylglycopeptide alpha-1,3-galactosyltransferase activity, UDP-Gal:Gal-beta-1->4GlcNAc-R alpha-1->3-galactosyltransferase activity, UDP-Gal:Galbeta1->4GlcNAc-R alpha1->3-galactosyltransferase activity, UDP-Gal:N-acetyllactosaminide alpha(1,3)-galactosyltransferase activity, UDP-Gal:N-acetyllactosaminide alpha-(1,3)-galactosyltransferase activity, UDP-Gal:N-acetyllactosaminide alpha-1,3-D-galactosyltransferase activity, UDP-Gal:beta-D-Gal(1,4)-D-GlcNAc alpha(1,3)-galactosyltransferase activity, UDP-Gal:beta-D-Gal(1,4)-D-GlcNAc alpha-(1,3)-galactosyltransferase activity, UDP-galactose-acetyllactosamine alpha-D-galactosyltransferase activity, UDP-galactose:N-acetyllactosaminide 3-alpha-D-galactosyltransferase activity, UDPgalactose:beta-D-galactosyl-beta-1,4-N-acetyl-D-glucosaminyl-glycopeptide alpha-1,3-D-galactosyltransferase activity, alpha-galactosyltransferase activity, beta-D-galactosyl-N-acetylglucosaminylglycopeptide alpha-1,3-galactosyltransferase activity, glucosaminylglycopeptide alpha-1,3-galactosyltransferase activity, uridine diphosphogalactose-acetyllactosamine alpha-1->3-galactosyltransferase activity, uridine diphosphogalactose-acetyllactosamine alpha1->3-galactosyltransferase activity, uridine diphosphogalactose-acetyllactosamine galactosyltransferase activity, uridine diphosphogalactose-galactosylacetylglucosaminylgalactosyl-glucosylceramide galactosyltransferase activity, uridine diphosphogalactose-galactosylacetylglucosaminylgalactosylglucosylceramide galactosyltransferase activity Relationships: is a type of UDP-galactosyltransferase activity [GO:0035250]